{
  "term_id": "GO:0003712",
  "term_label": "transcription coregulator activity",
  "gene_symbol": "LDB2",
  "gene": "UniProtKB:O43679",
  "gene_name": "LIM domain-binding protein 2"
}